extracellularly glycine-gated chloride channel activity [GO:0016934] (molecular function) Relationships: is a type of GO:0005237; is a type of GO:0005254; is a type of extracellularly glycine-gated ion channel activity [GO:0016933]; is a type of ligand-gated monoatomic anion channel activity [GO:0099095] Also known as: glycine receptor, extracellular-glycine-gated chloride channel activity, glycine-inhibited chloride channel activity Definition: Enables the transmembrane transfer of a chloride ion by a channel that opens when glycine is bound by the channel complex or one of its constituent parts on the extracellular side of the plasma membrane. Sources: GOC:mtg_transport, ISBN:0815340729